{
  "term_id": "UNKNOWN:0003",
  "gene": "UniProtKB:Q9NWD8",
  "gene_name": "Transmembrane protein 248",
  "gene_symbol": "TMEM248",
  "term_label": "Unknown cellular component"
}